soluble molecule recognition [GO:0009995] (biological process) Sources: GOC:go_curators Definition: The recognition of soluble molecules in the environment. Relationships: is a type of GO:0009593